{
  "gene": "UniProtKB:P22492",
  "term_id": "GO:0045910",
  "gene_symbol": "H1-6",
  "gene_name": "Histone H1t",
  "term_label": "negative regulation of DNA recombination"
}